{
  "term_id": "GO:0034657",
  "gene": "UniProtKB:Q96G75",
  "term_label": "GID complex",
  "gene_name": "E3 ubiquitin-protein transferase RMND5B",
  "gene_symbol": "RMND5B"
}